{
  "gene_symbol": "CCDC92",
  "gene": "UniProtKB:Q53HC0",
  "gene_name": "Coiled-coil domain-containing protein 92",
  "term_id": "UNKNOWN:0001",
  "term_label": "Unknown molecular function"
}